{
  "gene_symbol": "DSC2",
  "gene_name": "Desmocollin-2",
  "term_label": "calcium ion binding",
  "gene": "UniProtKB:Q02487",
  "term_id": "GO:0005509"
}